regulation of amino acid transport [GO:0051955] (biological process) Definition: Any process that modulates the frequency, rate or extent of the directed movement of amino acids into, out of or within a cell, or between cells, by means of some agent such as a transporter or pore. Subtypes: GO:0014048, GO:0014052, GO:0051941, negative regulation of amino acid transport [GO:0051956], positive regulation of amino acid transport [GO:0051957], regulation of proline transport [GO:0070881], regulation of amino acid transmembrane transport [GO:1903789], regulation of aspartate secretion [GO:1904448], regulation of glycine secretion, neurotransmission [GO:1904624], regulation of glutamine transport [GO:2000485] Relationships: is a type of regulation of amine transport [GO:0051952]; regulates amino acid transport [GO:0006865] Sources: GOC:ai